peroxisome-endoplasmic reticulum membrane tether activity [GO:0160229] (molecular function) Relationships: is a type of endoplasmic reticulum-organelle membrane tether activity [GO:0170009] Definition: The binding activity of a molecule that brings together a peroxisome and an ER membrane, either via membrane lipid binding or by interacting with a membrane protein. References: PMID:39271061